(1->3)-beta-D-glucan biosynthetic process [GO:0006075] (biological process) Definition: The chemical reactions and pathways resulting in the formation of (1->3)-beta-D-glucans, compounds composed of glucose residues linked by (1->3)-beta-D-glucosidic bonds. Sources: GOC:ai Also known as: 1,3-beta-D-glucan biosynthetic process, 1,3-beta-glucan anabolism, 1,3-beta-glucan biosynthesis, 1,3-beta-glucan formation, 1,3-beta-glucan synthesis, beta-1,3 glucan anabolism, beta-1,3 glucan biosynthesis, beta-1,3 glucan biosynthetic process, beta-1,3 glucan formation, beta-1,3 glucan synthesis Relationships: is a type of (1->3)-beta-D-glucan metabolic process [GO:0006074]; is_a GO:0051274 Subtypes: cell wall (1->3)-beta-D-glucan biosynthetic process [GO:0034411] Regulation: regulated by regulation of (1->3)-beta-D-glucan biosynthetic process [GO:0032953]; positively regulated by GO:0060635; negatively regulated by negative regulation of (1->3)-beta-D-glucan biosynthetic process [GO:0060636]